beta-pinacene synthase activity [GO:0106100] (molecular function) References: PMID:28696553 Sources: GOC:rjd Definition: Catalysis of the cyclization of geranylgeranyl pyrophosphate (GGPP) to yield the monocyclic diterpene beta-pinacene. Relationships: is a type of terpene synthase activity [GO:0010333]